{
  "term_label": "respiratory chain complex IV",
  "gene_name": "Normal mucosa of esophagus-specific gene 1 protein",
  "gene": "UniProtKB:Q9C002",
  "term_id": "GO:0045277",
  "gene_symbol": "NMES1"
}